{
  "gene_name": "Cerebellin-1",
  "gene": "UniProtKB:P23435",
  "term_id": "GO:0005615",
  "term_label": "extracellular space",
  "gene_symbol": "CBLN1"
}